{
  "term_label": "Unknown biological process",
  "gene": "UniProtKB:Q8N7P1",
  "gene_name": "Inactive phospholipase D5",
  "term_id": "UNKNOWN:0002",
  "gene_symbol": "PLD5"
}